{
  "term_label": "RNA polymerase II cis-regulatory region sequence-specific DNA binding",
  "gene": "UniProtKB:Q8IVH2",
  "gene_symbol": "FOXP4",
  "gene_name": "Forkhead box protein P4",
  "term_id": "GO:0000978"
}